{
  "term_id": "GO:0006367",
  "gene_symbol": "CDK7",
  "gene_name": "Cyclin-dependent kinase 7",
  "gene": "UniProtKB:P50613",
  "term_label": "transcription initiation at RNA polymerase II promoter"
}